{
  "term_label": "nucleus",
  "term_id": "GO:0005634",
  "gene_symbol": "H2AZ1",
  "gene": "UniProtKB:P0C0S5",
  "gene_name": "Histone H2A.Z"
}